{
  "gene": "UniProtKB:P20333",
  "term_label": "regulation of T cell proliferation",
  "gene_name": "Tumor necrosis factor receptor superfamily member 1B",
  "term_id": "GO:0042129",
  "gene_symbol": "TNFRSF1B"
}